{
  "term_id": "UNKNOWN:0003",
  "gene_name": "Testis-specific protein LINC02914",
  "term_label": "Unknown cellular component",
  "gene_symbol": "LINC02914",
  "gene": "UniProtKB:Q52M58"
}